sexual sporulation resulting in formation of a cellular spore [GO:0043935] (biological process) Definition: The formation of spores derived from the products of meiosis. A cellular spore is a cell form that can be used for dissemination, for survival of adverse conditions because of its heat and desiccation resistance, and/or for reproduction. Sources: GOC:pamgo_curators Relationships: is a type of sporulation resulting in formation of a cellular spore [GO:0030435]; is a type of sexual sporulation [GO:0034293] Subtypes: ascospore formation [GO:0030437], basidiospore formation [GO:0034295], zygospore formation [GO:0034296], oospore formation [GO:0075243] Regulation: regulated by regulation of sexual sporulation resulting in formation of a cellular spore [GO:0043940]; positively regulated by positive regulation of sexual sporulation resulting in formation of a cellular spore [GO:0043941]; negatively regulated by negative regulation of sexual sporulation resulting in formation of a cellular spore [GO:0043942]